{
  "gene": "UniProtKB:Q02127",
  "term_id": "GO:0005743",
  "term_label": "mitochondrial inner membrane",
  "gene_name": "Dihydroorotate dehydrogenase (quinone), mitochondrial",
  "gene_symbol": "DHODH"
}